photorespiration [GO:0009853] (biological process) Also known as: photorespiratory pathway Regulation: regulated by regulation of photorespiration [GO:0080093] Relationships: is a type of metabolic compound salvage [GO:0043094] Sources: ISBN:0198506732 Definition: A light-dependent catabolic process occurring concomitantly with photosynthesis in plants (especially C3 plants) whereby dioxygen (O2) is consumed and carbon dioxide (CO2) is evolved. The substrate is glycolate formed in large quantities in chloroplasts from 2-phosphoglycolate generated from ribulose 1,5-bisphosphate by the action of ribulose-bisphosphate carboxylase; the glycolate enters the peroxisomes where it is converted by glycolate oxidase to glyoxylate which undergoes transamination to glycine. This then passes into the mitochondria where it is decarboxylated forming one molecule of serine for every two molecules of glycine. This pathway also exists in photosynthetic bacteria.